3'-nucleotidase activity [GO:0008254] (molecular function) Sources: EC:3.1.3.6 Also known as: 3' nucleotidase activity, 3'-mononucleotidase activity, 3'-phosphatase activity, 3'-ribonucleotidase activity, 3'-ribonucleotide phosphohydrolase activity Definition: Catalysis of the reaction: a 3'-ribonucleotide + H2O = a ribonucleoside + phosphate. Relationships: is a type of nucleotidase activity [GO:0008252]